{
  "gene_symbol": "ZNF570",
  "term_id": "GO:0006357",
  "gene": "UniProtKB:Q96NI8",
  "term_label": "regulation of transcription by RNA polymerase II",
  "gene_name": "Zinc finger protein 570"
}